galactosamine transmembrane transporter activity [GO:0019196] (molecular function) Subtypes: N-acetylgalactosamine transmembrane transporter activity [GO:0015571], protein-N(PI)-phosphohistidine-galactosamine phosphotransferase system transporter activity [GO:0022876] Definition: Enables the transfer of galactosamine from one side of a membrane to the other. Galactosamine is an aminodeoxysugar; D-galactosamine is a constituent of some glycolipids and glycosaminoglycans, commonly as its N-acetyl derivative. Sources: GOC:mtg_transport, ISBN:0198506732, ISBN:0815340729 Relationships: is_a carbohydrate derivative transmembrane transporter activity [GO:1901505] Also known as: galactosamine porter activity